{
  "gene_symbol": "BRMS1L",
  "term_id": "GO:0000122",
  "gene": "UniProtKB:Q5PSV4",
  "gene_name": "Breast cancer metastasis-suppressor 1-like protein",
  "term_label": "negative regulation of transcription by RNA polymerase II"
}